{
  "gene_name": "Large ribosomal subunit protein P2",
  "gene": "UniProtKB:P05387",
  "gene_symbol": "RPLP2",
  "term_id": "UNKNOWN:0002",
  "term_label": "Unknown biological process"
}